mitotic nuclear envelope segregation [GO:0160052] (biological process) Definition: The mitotic cell cycle process in which the nuclear envelope, including nuclear pores, is equally distributed to the two daughter cells during the mitotic cell cycle. References: PMID:24184107 Sources: GOC:vw Relationships: is a type of mitotic cell cycle process [GO:1903047]; is part of mitotic nuclear division [GO:0140014]